positive regulation of dendrite extension [GO:1903861] (biological process) Note: An example of this is Mul1 in mouse (UniProt ID Q8VCM5) in PMID:24898855 inferred from mutant phenotype. Also known as: up regulation of dendrite extension, up-regulation of dendrite extension, upregulation of dendrite extension, activation of dendrite extension Relationships: is a type of positive regulation of cell growth [GO:0030307]; is a type of positive regulation of developmental growth [GO:0048639]; is a type of regulation of dendrite extension [GO:1903859]; positively regulates dendrite extension [GO:0097484] Definition: Any process that activates or increases the frequency, rate or extent of dendrite extension. References: PMID:24898855 Sources: GOC:PARL, GOC:TermGenie, GOC:pad, GO_REF:0000058